canonical inflammasome complex [GO:0061702] (cellular component) Definition: A cytosolic protein complex that is capable of activating caspase-1. Relationships: is_a protein-containing complex [GO:0032991]; is part of cytosol [GO:0005829] Subtypes: IPAF inflammasome complex [GO:0072557], NLRP1 inflammasome complex [GO:0072558], NLRP3 inflammasome complex [GO:0072559], AIM2 inflammasome complex [GO:0097169], CARD8 inflammasome complex [GO:0140634], NLRP6 inflammasome complex [GO:0140738] References: PMID:17599095 Sources: GOC:dph